pyridoxine transport [GO:0031923] (biological process) Relationships: is a type of organic hydroxy compound transport [GO:0015850]; is a type of GO:0031919 Subtypes: pyridoxine transmembrane transport [GO:1903092] Definition: The directed movement of pyridoxine into, out of or within a cell, or between cells, by means of some agent such as a transporter or pore. Pyridoxine, 2-methyl-3-hydroxy-4,5-bis(hydroxymethyl)pyridine, is one of the vitamin B6 compounds. Pyridoxal, pyridoxamine and pyridoxine are collectively known as vitamin B6, and are efficiently converted to the biologically active form of vitamin B6, pyridoxal phosphate. Sources: GOC:mah